{
  "gene_name": "EvC complex member EVC",
  "term_id": "UNKNOWN:0001",
  "term_label": "Unknown molecular function",
  "gene_symbol": "EVC",
  "gene": "UniProtKB:P57679"
}